{
  "gene_name": "Parkin coregulated gene protein",
  "gene_symbol": "PACRG",
  "term_id": "GO:0030544",
  "term_label": "Hsp70 protein binding",
  "gene": "UniProtKB:Q96M98"
}